{
  "term_id": "GO:0006641",
  "gene_symbol": "GK5",
  "term_label": "triglyceride metabolic process",
  "gene_name": "Putative glycerol kinase 5",
  "gene": "UniProtKB:Q6ZS86"
}